{
  "gene_symbol": "ADGRG1",
  "gene": "UniProtKB:Q9Y653",
  "term_id": "GO:0008201",
  "gene_name": "Adhesion G-protein coupled receptor G1",
  "term_label": "heparin binding"
}